{
  "gene_name": "Insulin-like growth factor-binding protein 3",
  "gene": "UniProtKB:P17936",
  "term_id": "GO:0031994",
  "gene_symbol": "IGFBP3",
  "term_label": "insulin-like growth factor I binding"
}